{
  "term_id": "GO:0000981",
  "gene_symbol": "ZNF761",
  "gene": "UniProtKB:Q86XN6",
  "term_label": "DNA-binding transcription factor activity, RNA polymerase II-specific",
  "gene_name": "Zinc finger protein 761"
}